{
  "term_label": "renal protein absorption",
  "gene_symbol": "AMN",
  "gene": "UniProtKB:Q9BXJ7",
  "term_id": "GO:0097017",
  "gene_name": "Protein amnionless"
}